{
  "term_label": "phosphatidylcholine-sterol O-acyltransferase activity",
  "gene": "UniProtKB:P04180",
  "term_id": "GO:0004607",
  "gene_symbol": "LCAT",
  "gene_name": "Phosphatidylcholine-sterol acyltransferase"
}